{
  "gene_name": "FAS-associated factor 2",
  "gene": "UniProtKB:Q96CS3",
  "term_id": "GO:0043130",
  "term_label": "ubiquitin binding",
  "gene_symbol": "FAF2"
}